{
  "gene": "UniProtKB:Q9BSA9",
  "gene_name": "Endosomal_lysosomal proton channel TMEM175",
  "gene_symbol": "TMEM175",
  "term_label": "lysosome",
  "term_id": "GO:0005764"
}